{
  "gene_name": "Caskin-1",
  "term_id": "GO:0007165",
  "gene_symbol": "CASKIN1",
  "gene": "UniProtKB:Q8WXD9",
  "term_label": "signal transduction"
}